{
  "gene_symbol": "RGP1",
  "gene": "UniProtKB:Q92546",
  "gene_name": "RAB6A-GEF complex partner protein 2",
  "term_label": "retrograde transport, endosome to Golgi",
  "term_id": "GO:0042147"
}